{
  "gene": "UniProtKB:Q8IY57",
  "term_label": "transcription coregulator activity",
  "gene_name": "YY1-associated factor 2",
  "gene_symbol": "YAF2",
  "term_id": "GO:0003712"
}